{
  "gene": "UniProtKB:Q9Y5N1",
  "gene_symbol": "HRH3",
  "term_id": "GO:0007197",
  "gene_name": "Histamine H3 receptor",
  "term_label": "adenylate cyclase-inhibiting G protein-coupled acetylcholine receptor signaling pathway"
}